{
  "term_label": "cholesterol metabolic process",
  "gene_symbol": "CH25H",
  "term_id": "GO:0008203",
  "gene_name": "Cholesterol 25-hydroxylase",
  "gene": "UniProtKB:O95992"
}